rRNA 5'-end processing [GO:0000967] (biological process) Sources: GOC:krc Definition: Any process involved in forming the mature 5' end of an rRNA molecule. Subtypes: exonucleolytic trimming to generate mature 5'-end of 5.8S rRNA from tricistronic rRNA transcript (SSU-rRNA, 5.8S rRNA, LSU-rRNA) [GO:0000465], endonucleolytic cleavage to generate mature 5'-end of SSU-rRNA from (SSU-rRNA, 5.8S rRNA, LSU-rRNA) [GO:0000472], generation of mature 5'-end of LSU-rRNA from tricistronic rRNA transcript (SSU-rRNA, 5.8S rRNA, LSU-rRNA) [GO:0000477] Also known as: rRNA 5' end processing Relationships: is a type of RNA 5'-end processing [GO:0000966]; is a type of rRNA processing [GO:0006364]